{
  "term_label": "adaptive immune response",
  "gene": "UniProtKB:P43405",
  "gene_name": "Tyrosine-protein kinase SYK",
  "term_id": "GO:0002250",
  "gene_symbol": "SYK"
}